{
  "gene_name": "Zinc finger protein 19",
  "term_id": "GO:0006357",
  "term_label": "regulation of transcription by RNA polymerase II",
  "gene_symbol": "ZNF19",
  "gene": "UniProtKB:P17023"
}